{
  "gene": "UniProtKB:P11137",
  "term_id": "GO:0008017",
  "gene_symbol": "MAP2",
  "term_label": "microtubule binding",
  "gene_name": "Microtubule-associated protein 2"
}